{
  "gene_name": "Hypocretin neuropeptide precursor",
  "gene": "UniProtKB:O43612",
  "term_label": "type 1 orexin receptor binding",
  "term_id": "GO:0031771",
  "gene_symbol": "HCRT"
}